{
  "gene": "UniProtKB:Q30KQ7",
  "term_id": "UNKNOWN:0001",
  "term_label": "Unknown molecular function",
  "gene_name": "Beta-defensin 113",
  "gene_symbol": "DEFB113"
}